{
  "gene": "UniProtKB:Q15036",
  "term_label": "early endosome",
  "gene_symbol": "SNX17",
  "term_id": "GO:0005769",
  "gene_name": "Sorting nexin-17"
}